nuclear stress granule [GO:0097165] (cellular component) References: PMID:10359787, PMID:12865437 Sources: GOC:ans Definition: A dense aggregation in the nucleus composed of proteins and RNAs that appear when the cell is under stress. Relationships: is a type of nuclear ribonucleoprotein granule [GO:0140168]